{
  "gene": "UniProtKB:Q9UIL1",
  "term_id": "UNKNOWN:0001",
  "gene_name": "Short coiled-coil protein",
  "gene_symbol": "SCOC",
  "term_label": "Unknown molecular function"
}